{
  "term_id": "GO:0008526",
  "gene_symbol": "PITPNA",
  "gene": "UniProtKB:Q00169",
  "gene_name": "Phosphatidylinositol transfer protein alpha isoform",
  "term_label": "phosphatidylinositol transfer activity"
}